{
  "term_label": "microtubule binding",
  "gene_name": "Centromere-associated protein E",
  "term_id": "GO:0008017",
  "gene_symbol": "CENPE",
  "gene": "UniProtKB:Q02224"
}